{
  "gene": "UniProtKB:Q6UB28",
  "term_id": "GO:0070006",
  "gene_name": "Methionine aminopeptidase 1D, mitochondrial",
  "term_label": "metalloaminopeptidase activity",
  "gene_symbol": "METAP1D"
}